{
  "gene": "UniProtKB:Q8N6L0",
  "gene_name": "Protein KASH5",
  "term_label": "nuclear outer membrane",
  "term_id": "GO:0005640",
  "gene_symbol": "KASH5"
}